{
  "gene": "UniProtKB:Q0VDI3",
  "gene_symbol": "TMEM267",
  "gene_name": "Transmembrane protein 267",
  "term_label": "Unknown cellular component",
  "term_id": "UNKNOWN:0003"
}